{
  "gene_name": "Protein pitchfork",
  "gene_symbol": "CIMAP3",
  "gene": "UniProtKB:Q8TCI5",
  "term_label": "regulation of cell projection organization",
  "term_id": "GO:0031344"
}